{
  "term_label": "Unknown cellular component",
  "gene_symbol": "LINC00311",
  "term_id": "UNKNOWN:0003",
  "gene": "UniProtKB:Q8N616",
  "gene_name": "Putative uncharacterized protein encoded by LINC00311"
}